{
  "term_label": "regulation of transcription by RNA polymerase II",
  "gene_name": "Zinc finger protein 345",
  "gene_symbol": "ZNF345",
  "term_id": "GO:0006357",
  "gene": "UniProtKB:Q14585"
}